{
  "gene_symbol": "APOBEC3H",
  "gene_name": "DNA dC-dU-editing enzyme APOBEC-3H",
  "term_id": "GO:0051607",
  "term_label": "defense response to virus",
  "gene": "UniProtKB:Q6NTF7"
}